{
  "gene": "UniProtKB:Q9NPD3",
  "gene_symbol": "EXOSC4",
  "gene_name": "Exosome complex component RRP41",
  "term_id": "GO:0000177",
  "term_label": "cytoplasmic exosome (RNase complex)"
}